{
  "gene_symbol": "RRP1",
  "gene_name": "Ribosomal RNA processing protein 1 homolog A",
  "term_label": "regulation of transcription by RNA polymerase II",
  "term_id": "GO:0006357",
  "gene": "UniProtKB:P56182"
}